{
  "gene_symbol": "NAT9",
  "gene": "UniProtKB:Q9BTE0",
  "term_id": "UNKNOWN:0003",
  "term_label": "Unknown cellular component",
  "gene_name": "Alpha_beta-tubulin-N-acetyltransferase 9"
}